{
  "gene_symbol": "CIDEC",
  "gene": "UniProtKB:Q96AQ7",
  "gene_name": "Lipid transferase CIDEC",
  "term_label": "lipid transfer activity",
  "term_id": "GO:0120013"
}